ATPase activity, coupled to transmembrane movement of ions, rotational mechanism [GO:0044769] (molecular function) Relationships: is a type of GO:0042625 Sources: GOC:jl Definition: Enables the transfer of ions from one side of a membrane to the other according to the reaction: ATP + H2O + ion(in) = ADP + phosphate + ion(out), by a rotational mechanism. Subtypes: proton-transporting ATPase activity, rotational mechanism [GO:0046961], sodium-transporting ATPase activity, rotational mechanism [GO:0046962]